{
  "gene": "UniProtKB:O60741",
  "term_id": "GO:0003254",
  "gene_symbol": "HCN1",
  "term_label": "regulation of membrane depolarization",
  "gene_name": "Potassium_sodium hyperpolarization-activated cyclic nucleotide-gated channel 1"
}